{
  "term_label": "establishment or maintenance of cell polarity",
  "term_id": "GO:0007163",
  "gene": "UniProtKB:Q5VZ46",
  "gene_symbol": "KIAA1614",
  "gene_name": "Uncharacterized protein KIAA1614"
}